{
  "gene_symbol": "C4orf19",
  "gene": "UniProtKB:Q8IY42",
  "term_id": "UNKNOWN:0003",
  "gene_name": "Uncharacterized protein C4orf19",
  "term_label": "Unknown cellular component"
}